{
  "term_label": "endoplasmic reticulum membrane",
  "term_id": "GO:0005789",
  "gene_symbol": "DPM3",
  "gene_name": "Dolichol-phosphate mannosyltransferase subunit 3",
  "gene": "UniProtKB:Q9P2X0"
}